{
  "term_label": "mitochondrion",
  "term_id": "GO:0005739",
  "gene_name": "Phenylalanine--tRNA ligase, mitochondrial",
  "gene_symbol": "FARS2",
  "gene": "UniProtKB:O95363"
}